{
  "term_label": "Unknown molecular function",
  "term_id": "UNKNOWN:0001",
  "gene": "UniProtKB:P06127",
  "gene_name": "T-cell surface glycoprotein CD5",
  "gene_symbol": "CD5"
}